{
  "term_label": "recycling endosome",
  "gene_symbol": "RAB4A",
  "term_id": "GO:0055037",
  "gene": "UniProtKB:P20338",
  "gene_name": "Ras-related protein Rab-4A"
}